muscle hyperplasia [GO:0014900] (biological process) Regulation: regulated by regulation of muscle hyperplasia [GO:0014738]; positively regulated by positive regulation of muscle hyperplasia [GO:0014739]; negatively regulated by negative regulation of muscle hyperplasia [GO:0014740] Subtypes: smooth muscle hyperplasia [GO:0014806] Sources: GOC:mtg_muscle Definition: A muscle system process that results in an increase in cell number by cell division, often leading to an increase in the size of an organ. Relationships: is a type of muscle adaptation [GO:0043500]